negative regulation of pronephric nephron tubule development [GO:1900207] (biological process) References: PMID:9758706 Sources: GOC:TermGenie, GOC:bf Definition: Any process that stops, prevents or reduces the frequency, rate or extent of pronephric nephron tubule development. Relationships: is_a GO:0051093; is a type of regulation of pronephric nephron tubule development [GO:1900206]; negatively regulates pronephric nephron tubule development [GO:0039020] Also known as: down regulation of pronephric nephron tubule development, down-regulation of pronephric nephron tubule development, downregulation of pronephric nephron tubule development, inhibition of pronephric nephron tubule development